{
  "term_id": "GO:0004984",
  "term_label": "olfactory receptor activity",
  "gene": "UniProtKB:O95006",
  "gene_symbol": "OR2F2",
  "gene_name": "Olfactory receptor 2F2"
}